ventral surface of cell [GO:0061835] (cellular component) Definition: The surface of a migrating cell that is in contact with the substratum or cell layer. References: PMID:11598004 Relationships: is a type of GO:0110165; is part of cell surface [GO:0009986]